extracellular vesicle [GO:1903561] (cellular component) References: PMID:24769233 Sources: GOC:TermGenie, GOC:pm, GO_REF:0000064 Also known as: microparticle Definition: Any vesicle that is part of the extracellular region. Subtypes: bacterial outer membrane vesicle [GO:0061701], GO:0070062, prominosome [GO:0071914], apoptotic body [GO:0097189], GO:0097691, exopher [GO:0160014], GO:1990742 Relationships: is_a vesicle [GO:0031982]; is a type of GO:0065010